{
  "term_id": "GO:0000172",
  "gene": "UniProtKB:Q9BUL9",
  "gene_name": "Ribonuclease P protein subunit p25",
  "gene_symbol": "RPP25",
  "term_label": "ribonuclease MRP complex"
}